2-hydroxypyridine 5-monooxygenase activity [GO:0047546] (molecular function) Relationships: is a type of monooxygenase activity [GO:0004497]; is a type of GO:0016705 Definition: Catalysis of the reaction: 2-hydroxypyridine + AH(2) + O2 = 2,5-dihydroxypyridine + A + H2O. Sources: EC:1.14.99.26, RHEA:16973 Also known as: 2-hydroxypyridine oxygenase activity, 2-hydroxypyridine,hydrogen-donor:oxygen oxidoreductase (5-hydroxylating)